{
  "gene_symbol": "RNF111",
  "term_label": "SUMO polymer binding",
  "term_id": "GO:0032184",
  "gene": "UniProtKB:Q6ZNA4",
  "gene_name": "E3 ubiquitin-protein ligase Arkadia"
}